{
  "gene": "UniProtKB:P49815",
  "term_id": "GO:0030178",
  "term_label": "negative regulation of Wnt signaling pathway",
  "gene_name": "Tuberin",
  "gene_symbol": "TSC2"
}